positive regulation of natural killer cell mediated cytotoxicity [GO:0045954] (biological process) Definition: Any process that activates or increases the frequency, rate or extent of natural killer cell mediated cytotoxicity. Sources: GOC:add, ISBN:0781735149 Also known as: positive regulation of NK cell mediated cell death, positive regulation of NK cell mediated cell killing, positive regulation of NK cell mediated cytotoxicity, positive regulation of natural killer cell mediated cell death, positive regulation of natural killer cell mediated cell killing, up regulation of natural killer cell mediated cytotoxicity, up-regulation of natural killer cell mediated cytotoxicity, upregulation of natural killer cell mediated cytotoxicity, activation of natural killer cell mediated cytotoxicity, stimulation of natural killer cell mediated cytotoxicity, positive regulation of NK cell mediated cytolysis, positive regulation of natural killer cell mediated cytolysis Relationships: is a type of positive regulation of leukocyte mediated cytotoxicity [GO:0001912]; is a type of GO:0002717; is a type of regulation of natural killer cell mediated cytotoxicity [GO:0042269]; positively regulates natural killer cell mediated cytotoxicity [GO:0042267] Subtypes: positive regulation of natural killer cell mediated cytotoxicity directed against tumor cell target [GO:0002860], susceptibility to natural killer cell mediated cytotoxicity [GO:0042271], positive regulation of natural killer cell degranulation [GO:0043323]